bone morphogenesis [GO:0060349] (biological process) Relationships: is a type of animal organ morphogenesis [GO:0009887]; is part of skeletal system morphogenesis [GO:0048705]; is part of GO:0060348 Subtypes: GO:0060350, replacement bone morphogenesis [GO:0061971], membrane bone morphogenesis [GO:0061973], craniofacial suture closure [GO:0160048], intramembranous bone morphogenesis [GO:1904770] Definition: The process in which bones are generated and organized. Sources: GOC:dph